{
  "gene_name": "Zinc finger MYND domain-containing protein 19",
  "term_label": "Unknown biological process",
  "gene": "UniProtKB:Q96E35",
  "gene_symbol": "ZMYND19",
  "term_id": "UNKNOWN:0002"
}